{
  "term_id": "GO:0007548",
  "term_label": "sex differentiation",
  "gene_symbol": "DMRTB1",
  "gene": "UniProtKB:Q96MA1",
  "gene_name": "Doublesex- and mab-3-related transcription factor B1"
}